{
  "gene_symbol": "VPS26C",
  "term_id": "GO:0006886",
  "gene_name": "Vacuolar protein sorting-associated protein 26C",
  "gene": "UniProtKB:O14972",
  "term_label": "intracellular protein transport"
}